regulation of retrograde trans-synaptic signaling by endocanabinoid [GO:0099178] (biological process) Definition: Any process that modulates the frequency, rate or extent of retrograde trans-synaptic signaling by an endocannabinoid. Also known as: regulation of endocannabinoid-mediated retrograde trans-synaptic signaling Relationships: is_a regulation of trans-synaptic signaling [GO:0099177]; RO_0002211 retrograde trans-synaptic signaling by endocannabinoid [GO:0098921] References: PMID:15664177 Sources: GOC:dos